glucose-1-phosphatase activity [GO:0008877] (molecular function) Also known as: D-glucose-1-phosphate phosphohydrolase activity, alpha-D-glucose-1-phosphate phosphohydrolase activity Relationships: is a type of GO:0050308 Definition: Catalysis of the reaction: alpha-D-glucose 1-phosphate + H2O = D-glucose + phosphate. Sources: EC:3.1.3.10